lactate fermentation to propionate and acetate [GO:0019652] (biological process) Sources: GOC:jl, MetaCyc:PROPFERM-PWY Also known as: acrylate pathway, nonrandomizing pathway, propionate fermentation Relationships: is a type of propionate metabolic process [GO:0019541]; is a type of non-glycolytic fermentation [GO:0019662] Definition: The anaerobic enzymatic conversion of lactate to propionate, concomitant with the oxidation of lactate to acetate and CO2 and yielding energy in the form of adenosine triphosphate (ATP).